{
  "gene": "UniProtKB:O95486",
  "term_label": "COPII-coated vesicle cargo loading",
  "gene_name": "Protein transport protein Sec24A",
  "term_id": "GO:0090110",
  "gene_symbol": "SEC24A"
}